{
  "term_label": "nucleus",
  "gene_name": "Double homeobox protein 1",
  "term_id": "GO:0005634",
  "gene_symbol": "DUX1",
  "gene": "UniProtKB:O43812"
}